{
  "gene": "UniProtKB:A8MPX8",
  "gene_symbol": "PP2D1",
  "gene_name": "Protein phosphatase 2C-like domain-containing protein 1",
  "term_id": "GO:0005634",
  "term_label": "nucleus"
}